{
  "gene_symbol": "SIRT1",
  "term_label": "subtelomeric heterochromatin formation",
  "term_id": "GO:0031509",
  "gene": "UniProtKB:Q96EB6",
  "gene_name": "NAD-dependent protein deacetylase sirtuin-1"
}